regulation of Wnt signaling pathway, calcium modulating pathway [GO:0008591] (BP) Relationships: is a type of regulation of non-canonical Wnt signaling pathway [GO:2000050]; RO_0002211 Wnt signaling pathway, calcium modulating pathway [GO:0007223] Definition: Any process that modulates the frequency, rate or extent of the series of molecular signals initiated by binding of a Wnt protein to a receptor on the surface of the target cell where activated receptors leads to an increase in intracellular calcium and activation of protein kinase C (PKC). Sources: GOC:dph, GOC:go_curators, GOC:tb Subtypes: negative regulation of Wnt signaling pathway, calcium modulating pathway [GO:0045812], positive regulation of Wnt signaling pathway, calcium modulating pathway [GO:0045813] Also known as: regulation of Wnt receptor signaling pathway, calcium modulating pathway, regulation of Wnt-activated signaling pathway, calcium modulating pathway, regulation of frizzled-2 signaling pathway, regulation of frizzled-2 signalling pathway